{
  "gene_symbol": "NOC2L",
  "gene_name": "Nucleolar complex protein 2 homolog",
  "gene": "UniProtKB:Q9Y3T9",
  "term_label": "ribosomal large subunit biogenesis",
  "term_id": "GO:0042273"
}